{
  "gene_name": "Receptor tyrosine-protein kinase erbB-3",
  "gene_symbol": "ERBB3",
  "term_label": "receptor complex",
  "term_id": "GO:0043235",
  "gene": "UniProtKB:P21860"
}